{
  "term_id": "GO:0000981",
  "gene_symbol": "OTX1",
  "term_label": "DNA-binding transcription factor activity, RNA polymerase II-specific",
  "gene": "UniProtKB:P32242",
  "gene_name": "Homeobox protein OTX1"
}